{
  "term_label": "DNA-binding transcription factor activity, RNA polymerase II-specific",
  "gene_symbol": "ISX",
  "term_id": "GO:0000981",
  "gene": "UniProtKB:Q2M1V0",
  "gene_name": "Intestine-specific homeobox"
}